regulation of lipopolysaccharide-mediated signaling pathway [GO:0031664] (biological process) Sources: GOC:mah Relationships: is a type of regulation of response to biotic stimulus [GO:0002831]; is a type of regulation of signal transduction [GO:0009966]; is_a regulation of response to external stimulus [GO:0032101]; regulates GO:0031663 Definition: Any process that modulates the frequency, rate or extent of signaling in response to detection of lipopolysaccharide. Also known as: regulation of LPS-mediated signaling pathway, regulation of lipopolysaccharide-mediated signalling pathway Subtypes: negative regulation of lipopolysaccharide-mediated signaling pathway [GO:0031665], positive regulation of lipopolysaccharide-mediated signaling pathway [GO:0031666]